{
  "gene_name": "Ras GTPase-activating protein nGAP",
  "term_label": "Unknown cellular component",
  "term_id": "UNKNOWN:0003",
  "gene_symbol": "RASAL2",
  "gene": "UniProtKB:Q9UJF2"
}